{
  "gene_symbol": "FGG",
  "gene_name": "Fibrinogen gamma chain",
  "gene": "UniProtKB:P02679",
  "term_id": "GO:0005102",
  "term_label": "signaling receptor binding"
}